negative regulation of octopamine or tyramine signaling pathway [GO:2000126] (biological process) Definition: Any process that stops, prevents, or reduces the frequency, rate or extent of octopamine or tyramine signaling pathway. Relationships: is a type of GO:0045744; is a type of regulation of octopamine or tyramine signaling pathway [GO:2000125]; negatively regulates octopamine or tyramine signaling pathway [GO:0007211] Also known as: negative regulation of octopamine or tyramine signalling pathway, negative regulation of octopamine/tyramine signaling pathway Subtypes: negative regulation of octopamine signaling pathway [GO:2000129], negative regulation of tyramine signaling pathway [GO:2000132] Sources: GOC:mah